positive regulation of methane biosynthetic process from trimethylamine [GO:1900332] (biological process) Definition: Any process that activates or increases the frequency, rate or extent of methane biosynthetic process from trimethylamine. Also known as: up regulation of methane biosynthetic process from trimethylamine, up-regulation of methane biosynthetic process from trimethylamine, upregulation of methane biosynthetic process from trimethylamine, activation of methane biosynthetic process from trimethylamine Relationships: is a type of positive regulation of amine metabolic process [GO:0033240]; is a type of regulation of methane biosynthetic process from trimethylamine [GO:1900330]; is a type of GO:1901579; is_a GO:1901857; positively regulates methane biosynthetic process from trimethylamine [GO:2001130] Sources: GOC:TermGenie, GOC:mengo_curators